negative regulation of cleistothecium development [GO:0070797] (BP) Sources: GOC:mah Definition: Any process that stops, prevents, or reduces the frequency, rate or extent of cleistothecium development, a process that leads to the formation of a cleistothecium. The cleistothecium is a closed sexual fruiting body that contains ascospores in linear asci, characteristic of some filamentous Ascomycete fungi such as members of the genera Aspergillus and Emericella. Relationships: is a type of regulation of cleistothecium development [GO:0070796]; is_a negative regulation of sporocarp development involved in sexual reproduction [GO:1902059]; RO_0002212 cleistothecium development [GO:0070791]